'de novo' pyrimidine nucleobase biosynthetic process [GO:0006207] (biological process) Also known as: 'de novo' pyrimidine base anabolism, 'de novo' pyrimidine base biosynthesis, 'de novo' pyrimidine base biosynthetic process, 'de novo' pyrimidine base formation, 'de novo' pyrimidine base synthesis Relationships: is a type of pyrimidine nucleobase biosynthetic process [GO:0019856] Definition: The chemical reactions and pathways resulting in the formation of pyrimidine nucleobases, 1,3-diazine, organic nitrogenous bases, beginning with the synthesis of a pyrimidine ring from simpler precursors. Sources: GOC:mah, ISBN:0716720094